{
  "term_label": "retrograde transport, endosome to Golgi",
  "gene_name": "TBC1 domain family member 10B",
  "gene_symbol": "TBC1D10B",
  "term_id": "GO:0042147",
  "gene": "UniProtKB:Q4KMP7"
}